tRNA uridine(34) acetyltransferase activity [GO:0106261] (molecular function) Relationships: is a type of GO:0016407; is a type of catalytic activity, acting on a tRNA [GO:0140101] References: PMID:25151136, PMID:30733442 Sources: RHEA:61020 Definition: Catalysis of the reaction: acetyl-CoA + H2O + S-adenosyl-L-methionine + uridine(34) in tRNA = 5'-deoxyadenosine + carboxymethyluridine(34) in tRNA + CoA + 2 H+ + L-methionine.